{
  "gene_name": "Protein FAM110D",
  "term_label": "Unknown cellular component",
  "gene": "UniProtKB:Q8TAY7",
  "term_id": "UNKNOWN:0003",
  "gene_symbol": "FAM110D"
}